{
  "gene_symbol": "OAS1",
  "gene_name": "2'-5'-oligoadenylate synthase 1",
  "term_label": "nucleoplasm",
  "term_id": "GO:0005654",
  "gene": "UniProtKB:P00973"
}